{
  "gene": "UniProtKB:P57081",
  "term_id": "GO:0043527",
  "term_label": "tRNA methyltransferase complex",
  "gene_symbol": "WDR4",
  "gene_name": "tRNA (guanine-N(7)-)-methyltransferase non-catalytic subunit WDR4"
}